{
  "gene": "UniProtKB:P00751",
  "term_id": "GO:0009617",
  "gene_name": "Complement factor B",
  "term_label": "response to bacterium",
  "gene_symbol": "CFB"
}